{
  "gene_symbol": "ESYT3",
  "gene": "UniProtKB:A0FGR9",
  "gene_name": "Extended synaptotagmin-3",
  "term_label": "phosphatidylcholine binding",
  "term_id": "GO:0031210"
}